phosphatidylinositol 5-phosphate biosynthetic process [GO:1904563] (biological process) Relationships: is a type of phosphatidylinositol phosphate biosynthetic process [GO:0046854]; is a type of GO:1904562 References: PMID:23916588 Sources: GOC:PARL, GOC:TermGenie, GOC:autophagy, GOC:dph, GOC:pad Also known as: phosphatidylinositol 5-phosphate anabolism, phosphatidylinositol 5-phosphate biosynthesis, phosphatidylinositol 5-phosphate formation, phosphatidylinositol 5-phosphate synthesis Definition: The chemical reactions and pathways resulting in the formation of phosphatidylinositol 5-phosphate.